neuromuscular process controlling posture [GO:0050884] (biological process) Sources: GOC:dph, GOC:tb Also known as: regulation of posture Relationships: is a type of neuromuscular process [GO:0050905]; has part musculoskeletal movement [GO:0050881] Definition: Any process in which an organism voluntarily modulates its posture, the alignment of its anatomical parts.